dextrin transmembrane transporter activity [GO:0042957] (molecular function) Relationships: is a type of polysaccharide transmembrane transporter activity [GO:0015159]; is part of dextrin transport [GO:0042955] Subtypes: maltodextrin transmembrane transporter activity [GO:0042958] Sources: GOC:jl, GOC:vk Definition: Enables the transfer of dextrin, any one, or the mixture, of the intermediate polysaccharides formed during the hydrolysis of starch, which are dextrorotatory, soluble in water, and precipitable in alcohol, from one side of a membrane to the other.